{
  "gene_symbol": "PRM1",
  "gene_name": "Sperm protamine P1",
  "term_label": "Unknown cellular component",
  "term_id": "UNKNOWN:0003",
  "gene": "UniProtKB:P04553"
}